RSP5-BUL ubiquitin ligase complex [GO:1990306] (cellular component) Definition: A ubiquitin ligase complex consisting of RSP5 and BUL components. It polyubiquinates plasma membrane transporters and permeases, required for their endocytosis and subsequent degradation in the vacuole. BUL1 or BUL2, respectively, bind to the target protein, enabling ubiquitylation by Rsp5. Phosphorylation of BUL proteins results in binding to 14-3-3 proteins, protecting the permeases from down-regulation. References: PMID:9931424 Sources: GOC:bhm Also known as: RSP5-BUL1 complex, RSP5-BUL2 complex Note: This complex has been identified in Saccharomyces cerevisiae (P19812) - see PMID:9931424 Relationships: is a type of intracellular protein-containing complex [GO:0140535]; is_a transferase complex [GO:1990234]